{
  "gene": "UniProtKB:P52272",
  "term_label": "RNA binding",
  "gene_name": "Heterogeneous nuclear ribonucleoprotein M",
  "term_id": "GO:0003723",
  "gene_symbol": "HNRNPM"
}